{
  "term_label": "glutathione binding",
  "term_id": "GO:0043295",
  "gene_name": "Glutathione synthetase",
  "gene_symbol": "GSS",
  "gene": "UniProtKB:P48637"
}